{
  "gene_symbol": "KATNAL1",
  "term_id": "GO:0005737",
  "gene": "UniProtKB:Q9BW62",
  "term_label": "cytoplasm",
  "gene_name": "Katanin p60 ATPase-containing subunit A-like 1"
}